flavanone 2-hydroxylase activity [GO:0033771] (molecular function) Sources: EC:1.14.14.162, RHEA:57584 Definition: Catalysis of the reaction: a flavanone + O2 + reduced [NADPH--hemoprotein reductase] = a 2-hydroxyflavanone + H+ + H2O + oxidized [NADPH--hemoprotein reductase]. Also known as: licodione synthase activity Relationships: is a type of oxidoreductase activity, acting on paired donors, with incorporation or reduction of molecular oxygen, reduced flavin or flavoprotein as one donor, and incorporation of one atom of oxygen [GO:0016712]